{
  "term_id": "GO:0005886",
  "gene": "UniProtKB:Q9GZN6",
  "gene_symbol": "SLC6A16",
  "gene_name": "Orphan sodium- and chloride-dependent neurotransmitter transporter NTT5",
  "term_label": "plasma membrane"
}